{
  "term_label": "helicase activity",
  "term_id": "GO:0004386",
  "gene": "UniProtKB:Q8IY37",
  "gene_name": "Probable ATP-dependent RNA helicase DHX37",
  "gene_symbol": "DHX37"
}